{
  "term_label": "Unknown cellular component",
  "gene_symbol": "KRTAP20-1",
  "gene": "UniProtKB:Q3LI63",
  "term_id": "UNKNOWN:0003",
  "gene_name": "Keratin-associated protein 20-1"
}